{
  "gene": "UniProtKB:Q9H9B1",
  "gene_symbol": "EHMT1",
  "term_label": "histone H3K9 methyltransferase activity",
  "term_id": "GO:0046974",
  "gene_name": "Histone-lysine N-methyltransferase EHMT1"
}